{
  "term_id": "UNKNOWN:0003",
  "term_label": "Unknown cellular component",
  "gene_name": "Testis-expressed protein 9",
  "gene_symbol": "TEX9",
  "gene": "UniProtKB:Q8N6V9"
}